argininosuccinate metabolic process [GO:0000053] (biological process) Relationships: is a type of GO:0006575; is a type of tricarboxylic acid metabolic process [GO:0072350]; is a type of GO:0170033; is a type of non-proteinogenic amino acid metabolic process [GO:0170041] Definition: The chemical reactions and pathways involving argininosuccinate, 2-(N(omega)-arginino)succinate, an intermediate in the ornithine-urea cycle, where it is synthesized from citrulline and aspartate. Sources: ISBN:0198506732 Also known as: argininosuccinate metabolism